ribosome disassembly [GO:0032790] (BP) Definition: The disaggregation of a ribosome into its constituent components; includes the dissociation of ribosomal subunits. Sources: GOC:mah, GOC:vk Also known as: ribosome recycling, ribosome dissociation factor Relationships: is a type of organelle disassembly [GO:1903008] Subtypes: rescue of stalled ribosome [GO:0072344]